gamma-catenin-TCF7L2 complex [GO:0071665] (cellular component) Relationships: is a type of catenin-TCF7L2 complex [GO:0071664] Also known as: gamma-catenin-TCF4 complex, plakoglobin-TCF4 complex Definition: A protein complex that contains gamma-catenin and TCF7L2 (TCF4), binds to the TCF DNA motif within a promoter element, and is involved in the regulation of WNT target gene transcription. References: PMID:14661054 Sources: GOC:BHF, GOC:vk